{
  "gene_symbol": "NLRP2",
  "gene": "UniProtKB:Q9NX02",
  "term_id": "UNKNOWN:0001",
  "term_label": "Unknown molecular function",
  "gene_name": "NACHT, LRR and PYD domains-containing protein 2"
}